{
  "term_label": "calcium ion binding",
  "gene_name": "Grancalcin",
  "term_id": "GO:0005509",
  "gene": "UniProtKB:P28676",
  "gene_symbol": "GCA"
}